collagen type XXI trimer [GO:1990320] (CC) References: PMID:17876790 Relationships: is a type of FACIT collagen trimer [GO:0005593] Definition: A collagen homotrimer of alpha1(XXI) chains; type XXI collagen triple helices found in the extracellular matrix component of blood vessel walls and in the cytoplasm of cultured human aortic smooth muscle.